{
  "gene": "UniProtKB:P17931",
  "gene_name": "Galectin-3",
  "term_id": "GO:0050918",
  "gene_symbol": "LGALS3",
  "term_label": "positive chemotaxis"
}